postsynaptic modulation of chemical synaptic transmission [GO:0099170] (biological process) Definition: Any process, acting in the postsynapse that results in modulation of chemical synaptic transmission. Relationships: is a type of modulation of chemical synaptic transmission [GO:0050804]; BFO_0000066 postsynapse [GO:0098794] Subtypes: regulation of protein catabolic process at postsynapse, modulating synaptic transmission [GO:0099576], regulation of translation at postsynapse, modulating synaptic transmission [GO:0099578] Sources: GOC:dos